{
  "gene_name": "ATPase WRNIP1",
  "gene": "UniProtKB:Q96S55",
  "gene_symbol": "WRNIP1",
  "term_id": "GO:0005634",
  "term_label": "nucleus"
}